{
  "gene": "UniProtKB:Q6TDU7",
  "gene_name": "Dynein axonemal intermediate chain 7",
  "gene_symbol": "DNAI7",
  "term_id": "GO:0008017",
  "term_label": "microtubule binding"
}